{
  "term_label": "long-chain fatty acid binding",
  "gene_symbol": "FABP2",
  "gene": "UniProtKB:P12104",
  "gene_name": "Fatty acid-binding protein, intestinal",
  "term_id": "GO:0036041"
}